{
  "gene": "UniProtKB:Q9UBP5",
  "term_label": "Notch signaling pathway",
  "gene_name": "Hairy_enhancer-of-split related with YRPW motif protein 2",
  "gene_symbol": "HEY2",
  "term_id": "GO:0007219"
}